{
  "term_label": "Unknown cellular component",
  "term_id": "UNKNOWN:0003",
  "gene_symbol": "SGK2",
  "gene_name": "Serine_threonine-protein kinase Sgk2",
  "gene": "UniProtKB:Q9HBY8"
}